glycyl-radical enzyme activating activity [GO:0043364] (molecular function) References: PMID:24486374 Sources: GOC:jl Relationships: is a type of oxidoreductase activity [GO:0016491] Also known as: catalysis of free radical formation Definition: Catalyzes the activation of an enzyme by generating an organic free radical on a glycine residue via a homolytic cleavage of S-adenosyl-L-methionine (SAM). Subtypes: [formate-C-acetyltransferase]-activating enzyme activity [GO:0043365], [choline trimethylamine-lyase]-activating enzyme activity [GO:0140111]